{
  "gene_symbol": "ZNF573",
  "term_label": "RNA polymerase II cis-regulatory region sequence-specific DNA binding",
  "gene": "UniProtKB:Q86YE8",
  "gene_name": "Zinc finger protein 573",
  "term_id": "GO:0000978"
}